{
  "term_id": "GO:0005739",
  "term_label": "mitochondrion",
  "gene_symbol": "CHCHD6",
  "gene_name": "MICOS complex subunit MIC25",
  "gene": "UniProtKB:Q9BRQ6"
}